{
  "gene_symbol": "EEPD1",
  "gene_name": "Endonuclease_exonuclease_phosphatase family domain-containing protein 1",
  "gene": "UniProtKB:Q7L9B9",
  "term_id": "UNKNOWN:0002",
  "term_label": "Unknown biological process"
}